{
  "term_label": "clathrin adaptor activity",
  "gene": "UniProtKB:O94973",
  "gene_name": "AP-2 complex subunit alpha-2",
  "gene_symbol": "AP2A2",
  "term_id": "GO:0035615"
}